trans-cinnamate 4-monooxygenase activity [GO:0016710] (molecular function) Also known as: CA4H activity, cinnamate 4-hydroxylase activity, cinnamate 4-monooxygenase activity, cinnamate hydroxylase activity, cinnamic 4-hydroxylase activity, cinnamic acid 4-hydroxylase activity, cinnamic acid 4-monooxygenase activity, cinnamic acid p-hydroxylase activity, cytochrome P450 cinnamate 4-hydroxylase activity, hydroxylase, cinnamate 4-, oxygenase, cinnamate 4-mono-, t-cinnamic acid hydroxylase activity, trans-cinnamate 4-hydroxylase activity, trans-cinnamate,NADPH:oxygen oxidoreductase (4-hydroxylating), trans-cinnamic acid 4-hydroxylase activity Definition: Catalysis of the reaction: trans-cinnamate + NADPH + H+ + O2 = 4-hydroxycinnamate + NADP+ + H2O. Relationships: is a type of oxidoreductase activity, acting on paired donors, with incorporation or reduction of molecular oxygen, NAD(P)H as one donor, and incorporation of one atom of oxygen [GO:0016709] Sources: EC:1.14.14.91